{
  "term_label": "detection of chemical stimulus involved in sensory perception of bitter taste",
  "gene_symbol": "TAS2R5",
  "term_id": "GO:0001580",
  "gene_name": "Taste receptor type 2 member 5",
  "gene": "UniProtKB:Q9NYW4"
}